{
  "term_id": "UNKNOWN:0002",
  "term_label": "Unknown biological process",
  "gene_name": "Inter-alpha-trypsin inhibitor heavy chain H2",
  "gene_symbol": "ITIH2",
  "gene": "UniProtKB:P19823"
}